positive regulation of integrin biosynthetic process [GO:0045726] (biological process) Subtypes: GO:0045775 Definition: Any process that activates or increases the frequency, rate or extent of the chemical reactions and pathways resulting in the formation of integrins. Relationships: is a type of positive regulation of macromolecule biosynthetic process [GO:0010557]; is a type of regulation of integrin biosynthetic process [GO:0045113]; is a type of positive regulation of cellular component organization [GO:0051130]; positively regulates integrin biosynthetic process [GO:0045112] Also known as: positive regulation of integrin anabolism, positive regulation of integrin biosynthesis, positive regulation of integrin formation, positive regulation of integrin synthesis, up regulation of integrin biosynthetic process, up-regulation of integrin biosynthetic process, upregulation of integrin biosynthetic process, activation of integrin biosynthetic process, stimulation of integrin biosynthetic process Sources: GOC:go_curators